{
  "gene_name": "Carbonic anhydrase-related protein",
  "term_id": "UNKNOWN:0003",
  "gene_symbol": "CA8",
  "term_label": "Unknown cellular component",
  "gene": "UniProtKB:P35219"
}